{
  "gene": "UniProtKB:P46098",
  "term_id": "GO:0022850",
  "gene_name": "5-hydroxytryptamine receptor 3A",
  "term_label": "serotonin-gated monoatomic cation channel activity",
  "gene_symbol": "HTR3A"
}